anaerobic L-glutamate catabolic process [GO:0019670] (biological process) Sources: GOC:jl Subtypes: L-glutamate catabolic process via 2-hydroxyglutarate [GO:0019552] Relationships: is a type of GO:0006538; is a type of anaerobic amino acid catabolic process [GO:0019665] Definition: The anaerobic chemical reactions and pathways resulting in the breakdown of L-glutamate, yielding energy in the form of ATP. Also known as: glutamate fermentation